{
  "term_label": "aldose reductase (NADPH) activity",
  "gene_symbol": "AKR1C3",
  "gene": "UniProtKB:P42330",
  "gene_name": "Aldo-keto reductase family 1 member C3",
  "term_id": "GO:0004032"
}